{
  "gene_name": "CAP-Gly domain-containing linker protein 2",
  "term_label": "cell cortex",
  "gene_symbol": "CLIP2",
  "gene": "UniProtKB:Q9UDT6",
  "term_id": "GO:0005938"
}